{
  "gene_symbol": "KRTAP13-1",
  "gene": "UniProtKB:Q8IUC0",
  "gene_name": "Keratin-associated protein 13-1",
  "term_id": "UNKNOWN:0002",
  "term_label": "Unknown biological process"
}